{
  "gene_name": "Versican core protein",
  "gene": "UniProtKB:P13611",
  "term_label": "extracellular space",
  "term_id": "GO:0005615",
  "gene_symbol": "VCAN"
}